regulation of tumor necrosis factor-mediated signaling pathway [GO:0010803] (biological process) Definition: Any process that modulates the rate or extent of the tumor necrosis factor-mediated signaling pathway. The tumor necrosis factor-mediated signaling pathway is the series of molecular signals generated as a consequence of tumor necrosis factor binding to a cell surface receptor. Sources: GOC:dph, GOC:tb Also known as: regulation of TNF signaling, regulation of TNF-mediated signaling pathway, regulation of tumor necrosis factor-mediated signalling pathway Relationships: is a type of regulation of cytokine-mediated signaling pathway [GO:0001959]; regulates GO:0033209 Subtypes: negative regulation of tumor necrosis factor-mediated signaling pathway [GO:0010804], positive regulation of tumor necrosis factor-mediated signaling pathway [GO:1903265]